{
  "gene": "UniProtKB:O75964",
  "term_label": "Unknown cellular component",
  "term_id": "UNKNOWN:0003",
  "gene_symbol": "ATP5MG",
  "gene_name": "ATP synthase subunit g, mitochondrial"
}